dichotomous subdivision of prostate epithelial cord terminal unit [GO:0060524] (biological process) Definition: The process in which a prostate epithelial cord bifurcates at its end. Also known as: prostate epithelial cord bifurcation References: PMID:18977204 Sources: GOC:dph Relationships: is_a developmental process involved in reproduction [GO:0003006]; is a type of GO:0060600; is part of branching involved in prostate gland morphogenesis [GO:0060442]